amino acid transmembrane export from vacuole [GO:0032974] (biological process) Also known as: amino acid efflux from vacuole, vacuolar amino acid export Relationships: is a type of GO:0003333; is_a vacuolar transmembrane transport [GO:0034486] Definition: The directed movement of amino acids out of the vacuole, across the vacuolar membrane. Subtypes: basic amino acid transmembrane export from vacuole [GO:0034488], neutral amino acid transmembrane export from vacuole [GO:0034489], L-glutamate transmembrane export from vacuole [GO:0089704], L-ornithine transmembrane export from vacuole [GO:0089706], L-lysine transmembrane export from vacuole [GO:0089707], L-histidine transmembrane export from vacuole [GO:0089708], L-histidine transmembrane transport from lysosomal lumen to cytosol [GO:1904918], L-arginine transmembrane export from vacuole [GO:1990818] Sources: GOC:mah